{
  "gene": "UniProtKB:P01893",
  "gene_symbol": "HLA-H",
  "gene_name": "Putative HLA class I histocompatibility antigen, alpha chain H",
  "term_id": "GO:0009897",
  "term_label": "external side of plasma membrane"
}